interleukin-2 receptor activity [GO:0004911] (molecular function) Definition: Combining with interleukin-2 and transmitting the signal from one side of the membrane to the other to initiate a change in cell activity. Sources: GOC:jl, GOC:signaling Also known as: IL-2 receptor activity, IL-2R Relationships: is_a cytokine receptor activity [GO:0004896]; is part of interleukin-2-mediated signaling pathway [GO:0038110]; has part interleukin-2 binding [GO:0019976]